{
  "gene": "UniProtKB:Q9Y250",
  "gene_name": "Leucine zipper putative tumor suppressor 1",
  "term_id": "GO:0048167",
  "term_label": "regulation of synaptic plasticity",
  "gene_symbol": "LZTS1"
}